{
  "gene": "UniProtKB:Q12912",
  "term_id": "UNKNOWN:0001",
  "gene_symbol": "IRAG2",
  "gene_name": "Inositol 1,4,5-triphosphate receptor associated 2",
  "term_label": "Unknown molecular function"
}